{
  "gene": "UniProtKB:Q09MP3",
  "term_label": "Unknown biological process",
  "gene_symbol": "RAD51AP2",
  "gene_name": "RAD51-associated protein 2",
  "term_id": "UNKNOWN:0002"
}